flagellum attachment zone organization [GO:0110140] (biological process) Also known as: FAZ organization, flagellum attachment zone organisation Relationships: is a type of cell junction organization [GO:0034330] Definition: A process that is carried out at the cellular level which results in the assembly, arrangement of constituent parts, or disassembly of a flagellum attachment zone. FAZ is a network of cytoskeletal and membranous connections responsible for the lateral attachment of the cilium to the cell body in some trypanosomatid species. References: PMID:26776656 Sources: GOC:ach